isoquinoline alkaloid catabolic process [GO:0071274] (biological process) Relationships: is a type of alkaloid catabolic process [GO:0009822]; is_a isoquinoline alkaloid metabolic process [GO:0033076] Definition: The chemical reactions and pathways resulting in the breakdown of isoquinoline alkaloids, alkaloid compounds that contain bicyclic N-containing aromatic rings and are derived from a 3,4-dihydroxytyramine (dopamine) precursor that undergoes a Schiff base addition with aldehydes of different origin. Subtypes: morphine catabolic process [GO:0071273], codeine catabolic process [GO:2001292] References: PMID:23666088 Sources: GOC:mah Also known as: isoquinoline alkaloid breakdown, isoquinoline alkaloid catabolism, isoquinoline alkaloid degradation, ipecac alkaloid catabolism